{
  "gene_symbol": "CARD9",
  "term_id": "GO:0032449",
  "term_label": "CBM complex",
  "gene": "UniProtKB:Q9H257",
  "gene_name": "Caspase recruitment domain-containing protein 9"
}